{
  "gene_name": "Serine protease 27",
  "term_id": "GO:0008236",
  "term_label": "serine-type peptidase activity",
  "gene_symbol": "PRSS27",
  "gene": "UniProtKB:Q9BQR3"
}